{
  "term_label": "nucleus",
  "gene": "UniProtKB:Q8N3U4",
  "term_id": "GO:0005634",
  "gene_symbol": "STAG2",
  "gene_name": "Cohesin subunit SA-2"
}